{
  "term_label": "L-aspartate transmembrane transporter activity",
  "gene_symbol": "SLC1A5",
  "gene": "UniProtKB:Q15758",
  "term_id": "GO:0015183",
  "gene_name": "Neutral amino acid transporter B(0)"
}